3-phosphoglyceroyl-phosphate-polyphosphate phosphotransferase activity [GO:0047335] (molecular function) Sources: EC:2.7.4.17, MetaCyc:2.7.4.17-RXN Relationships: is a type of phosphotransferase activity, phosphate group as acceptor [GO:0016776] Definition: Catalysis of the reaction: long-chain-polyphosphate + 3-phospho-D-glyceroyl-phosphate = long-chain-polyphosphate + 3-phosphoglycerate. Also known as: 1,3-diphosphoglycerate-polyphosphate phosphotransferase activity, 3-phospho-D-glyceroyl-phosphate:polyphosphate phosphotransferase activity, diphosphoglycerate-polyphosphate phosphotransferase activity